{
  "gene_name": "Chondroitin sulfate synthase 1",
  "gene": "UniProtKB:Q86X52",
  "gene_symbol": "CHSY1",
  "term_id": "GO:0050650",
  "term_label": "chondroitin sulfate proteoglycan biosynthetic process"
}